{
  "gene": "UniProtKB:P52564",
  "gene_name": "Dual specificity mitogen-activated protein kinase kinase 6",
  "term_label": "MAP kinase kinase activity",
  "term_id": "GO:0004708",
  "gene_symbol": "MAP2K6"
}